negative regulation of oxidoreductase activity [GO:0051354] (biological process) Definition: Any process that stops or reduces the rate of oxidoreductase activity, the catalysis of an oxidation-reduction (redox) reaction, a reversible chemical reaction in which the oxidation state of an atom or atoms within a molecule is altered. Sources: GOC:ai Relationships: is a type of GO:0043086; is a type of regulation of oxidoreductase activity [GO:0051341]; negatively regulates oxidoreductase activity [GO:0016491] Also known as: down regulation of oxidoreductase activity, down-regulation of oxidoreductase activity, downregulation of oxidoreductase activity, oxidoreductase inhibitor, inhibition of oxidoreductase activity Subtypes: negative regulation of nitric-oxide synthase activity [GO:0051001]